{
  "gene_symbol": "TSPY8",
  "term_id": "UNKNOWN:0002",
  "gene_name": "Testis-specific Y-encoded protein 8",
  "term_label": "Unknown biological process",
  "gene": "UniProtKB:P0CW00"
}